{
  "term_id": "GO:0009897",
  "term_label": "external side of plasma membrane",
  "gene_name": "HERV-H LTR-associating protein 2",
  "gene": "UniProtKB:Q9UM44",
  "gene_symbol": "HHLA2"
}